{
  "term_label": "actin crosslink formation",
  "gene_name": "Brain-specific angiogenesis inhibitor 1-associated protein 2-like protein 1",
  "term_id": "GO:0051764",
  "gene": "UniProtKB:Q9UHR4",
  "gene_symbol": "BAIAP2L1"
}